{
  "gene_symbol": "CAGE1",
  "term_id": "UNKNOWN:0003",
  "term_label": "Unknown cellular component",
  "gene_name": "Cancer-associated gene 1 protein",
  "gene": "UniProtKB:Q8TC20"
}